germ cell migration [GO:0008354] (biological process) Sources: GOC:bf, GOC:jl Definition: The orderly movement of a cell specialized to produce haploid gametes through the embryo from its site of production to the place where the gonads will form. Relationships: is_a cell migration [GO:0016477]; is part of gamete generation [GO:0007276] Also known as: germ-cell migration, pole cell migration, primordial germ cell migration